{
  "gene_symbol": "FOXO3",
  "term_label": "RNA polymerase II cis-regulatory region sequence-specific DNA binding",
  "gene_name": "Forkhead box protein O3",
  "term_id": "GO:0000978",
  "gene": "UniProtKB:O43524"
}